phospholipase A2 activity [GO:0004623] (molecular function) Regulation: positively regulated by phospholipase A2 activator activity [GO:0016005]; negatively regulated by phospholipase A2 inhibitor activity [GO:0019834] Also known as: cytosolic phospholipase A2 activity, phospholipase A2 activity (consuming 1,2-dipalmitoylphosphatidylcholine), phospholipase A2 activity consuming 1,2-dioleoylphosphatidylethanolamine), secreted phospholipase A2 activity, lecithinase A activity, phosphatidase activity, phosphatidolipase activity, phosphatidylcholine 2-acylhydrolase activity Definition: Catalysis of the reaction: a 1,2-diacyl-sn-glycero-3-phospholipid + H2O = 1-acyl-sn-glycero-3-phospholipid + a fatty acid. This reaction removes the fatty acid attached to the sn2-position. Substrates include phosphatidylcholine, phosphatidylethanolamine, choline plasmalogen and phosphatides. Subtypes: calcium-dependent phospholipase A2 activity [GO:0047498], calcium-independent phospholipase A2 activity [GO:0047499] Relationships: is a type of phospholipase activity [GO:0004620]; is a type of carboxylic ester hydrolase activity [GO:0052689] Sources: RHEA:15801